{
  "term_id": "GO:0005829",
  "gene_symbol": "PRKACG",
  "gene_name": "cAMP-dependent protein kinase catalytic subunit gamma",
  "term_label": "cytosol",
  "gene": "UniProtKB:P22612"
}